host-symbiont bicellular tight junction [GO:0044647] (cellular component) Definition: An occluding cell-cell junction formed between the membranes of the apical end of an invading cell (e.g. a merozoite in Plasmodium) and a host target cell (e.g. erythrocyte for Plasmodium infection). The junction is a stable yet dynamic structure that moves around the symbiont cell during invasion, enclosing it in a vacuole surrounded by a membrane. Relationships: is a type of bicellular tight junction [GO:0005923] Also known as: host-parasite tight junction, host-pathogen tight junction References: PMID:21803641 Sources: GOC:jl